{
  "gene": "UniProtKB:A0A0A0MT76",
  "term_id": "UNKNOWN:0002",
  "term_label": "Unknown biological process",
  "gene_symbol": "IGLJ1",
  "gene_name": "Immunoglobulin lambda joining 1"
}